9,10 (9', 10')-carotenoid-cleaving dioxygenase activity [GO:0010437] (MF) Definition: Catalysis of the oxidative cleavage of carotenoids at the (9, 10) and/or (9', 10') double bond. Relationships: is a type of carotenoid dioxygenase activity [GO:0010436] References: PMID:16459333